hippocampal mossy fiber expansion [GO:1990026] (cellular component) Definition: Synaptic expansion of hippocampal mossy fiber axon that makes contact with the thorny excrescences of hippocampal CA3 pyramidal cell dendrites. Sources: NIF_Subcellular:nlx_subcell_1005002 Also known as: mossy fiber expansion, dentate gyrus granule cell axonal bouton, dentate gyrus mossy fiber expansion Relationships: is a type of GO:0043195; BFO_0000050 hippocampal mossy fiber [GO:0097457]